{
  "gene_name": "Palmitoyltransferase ZDHHC5",
  "gene_symbol": "ZDHHC5",
  "gene": "UniProtKB:Q9C0B5",
  "term_id": "GO:0062208",
  "term_label": "positive regulation of pattern recognition receptor signaling pathway"
}